membrane protein proteolysis involved in retrograde protein transport, ER to cytosol [GO:1904211] (biological process) References: PMID:22795130 Sources: GOC:PARL, GOC:TermGenie, GOC:bf, GO_REF:0000060 Also known as: intramembrane cleavage of ERAD substrate, intramembrane proteolysis involved in ERAD, membrane protein proteolysis involved in protein dislocation from ER, membrane protein proteolysis involved in protein retrotranslocation, ER to cytosol, membrane protein proteolysis involved in retrograde protein transport, endoplasmic reticulum to cytosol Definition: Any membrane protein proteolysis that is involved in retrograde protein transport, ER to cytosol. Relationships: is a type of membrane protein proteolysis [GO:0033619]; is a type of proteolysis involved in protein catabolic process [GO:0051603]; is part of retrograde protein transport, ER to cytosol [GO:0030970]